negative regulation of iridophore differentiation [GO:0050943] (biological process) Sources: GOC:ai Relationships: is a type of regulation of iridophore differentiation [GO:0050937]; is_a GO:0050941; negatively regulates iridophore differentiation [GO:0050935] Also known as: down regulation of iridophore differentiation, down-regulation of iridophore differentiation, downregulation of iridophore differentiation, inhibition of iridophore differentiation Definition: Any process that stops, prevents, or reduces the frequency, rate or extent of iridophore differentiation.